{
  "term_id": "GO:1990904",
  "gene_name": "Heterogeneous nuclear ribonucleoprotein U",
  "gene": "UniProtKB:Q00839",
  "term_label": "ribonucleoprotein complex",
  "gene_symbol": "HNRNPU"
}